{
  "gene_name": "Keratin, type II cytoskeletal 4",
  "term_label": "structural constituent of skin epidermis",
  "gene": "UniProtKB:P19013",
  "term_id": "GO:0030280",
  "gene_symbol": "KRT4"
}